{
  "gene_symbol": "DGCR6L",
  "gene": "UniProtKB:Q9BY27",
  "term_id": "UNKNOWN:0003",
  "gene_name": "Protein DGCR6L",
  "term_label": "Unknown cellular component"
}